feminization of hermaphroditic germ-line [GO:0040022] (biological process) Sources: GOC:ems Definition: The determination of female sex and sexual phenotype in the germ-line of the hermaphrodite. Relationships: is a type of GO:0040021